{
  "term_id": "UNKNOWN:0001",
  "gene_symbol": "OSGEPL1",
  "gene": "UniProtKB:Q9H4B0",
  "gene_name": "tRNA N6-adenosine threonylcarbamoyltransferase, mitochondrial",
  "term_label": "Unknown molecular function"
}